{
  "gene_symbol": "SGO1",
  "term_label": "mitotic cohesin complex",
  "gene_name": "Shugoshin 1",
  "term_id": "GO:0030892",
  "gene": "UniProtKB:Q5FBB7"
}